{
  "gene_symbol": "KLHDC8A",
  "term_id": "UNKNOWN:0001",
  "gene_name": "Kelch domain-containing protein 8A",
  "term_label": "Unknown molecular function",
  "gene": "UniProtKB:Q8IYD2"
}